negative regulation of protein localization to cell surface [GO:2000009] (biological process) Definition: Any process that stops, prevents, or reduces the frequency, rate or extent of protein localization to the cell surface. Sources: GOC:obol Also known as: negative regulation of protein localisation at cell surface, negative regulation of protein localization at cell surface Relationships: is_a negative regulation of protein localization [GO:1903828]; is a type of GO:2000008; negatively regulates protein localization to cell surface [GO:0034394]